positive regulation of platelet-derived growth factor production [GO:0090362] (biological process) Definition: Any process that increases the rate, frequency, or extent of the appearance of any platelet-derived growth factor due to biosynthesis or secretion following a cellular stimulus, resulting in an increase in its intracellular or extracellular levels. Sources: GOC:BHF Relationships: is a type of GO:0001819; is a type of regulation of platelet-derived growth factor production [GO:0090361]; positively regulates platelet-derived growth factor production [GO:0090360]